{
  "gene_symbol": "WIPF2",
  "term_id": "UNKNOWN:0003",
  "gene": "UniProtKB:Q8TF74",
  "term_label": "Unknown cellular component",
  "gene_name": "WAS_WASL-interacting protein family member 2"
}